erythrocyte development [GO:0048821] (biological process) Definition: The process whose specific outcome is the progression of an erythrocyte over time, from its formation to the mature structure. Sources: GOC:devbiol Also known as: RBC development, red blood cell development Relationships: is a type of GO:0061515; is part of erythrocyte differentiation [GO:0030218] Subtypes: enucleate erythrocyte development [GO:0048822], nucleate erythrocyte development [GO:0048823]